{
  "gene": "UniProtKB:Q8NEE0",
  "term_label": "Unknown cellular component",
  "gene_symbol": "KLHL30-AS1",
  "gene_name": "Putative uncharacterized protein KLHL30-AS1",
  "term_id": "UNKNOWN:0003"
}